macrophage migration inhibitory factor binding [GO:0035718] (MF) Definition: Binding to the cytokine, macrophage migration inhibitory factor. Relationships: is a type of cytokine binding [GO:0019955] Also known as: MIF binding References: PMID:19601712 Sources: GOC:BHF